{
  "gene_symbol": "CMTR2",
  "term_label": "nucleus",
  "term_id": "GO:0005634",
  "gene_name": "Cap-specific mRNA (nucleoside-2'-O-)-methyltransferase 2",
  "gene": "UniProtKB:Q8IYT2"
}